pre-replicative complex assembly involved in premeiotic DNA replication [GO:1902984] (biological process) Sources: GOC:TermGenie, GO_REF:0000060 Definition: Any pre-replicative complex assembly involved in meiotic cell cycle DNA replication. Also known as: pre-RC complex assembly involved in meiosis, pre-replicative complex assembly involved in meiosis, pre-replicative complex formation involved in meiosis, nuclear pre-replicative complex assembly involved in meiotic cell cycle, pre-replicative complex assembly involved in meiotic cell cycle DNA replication Relationships: is a type of pre-replicative complex assembly involved in nuclear cell cycle DNA replication [GO:0006267]; is_a meiotic cell cycle process [GO:1903046]; is part of premeiotic DNA replication [GO:0006279]